{
  "gene_symbol": "C5orf46",
  "gene_name": "Uncharacterized protein C5orf46",
  "term_id": "UNKNOWN:0001",
  "gene": "UniProtKB:Q6UWT4",
  "term_label": "Unknown molecular function"
}